{
  "gene_symbol": "COPG2",
  "term_label": "endoplasmic reticulum",
  "gene": "UniProtKB:Q9UBF2",
  "gene_name": "Coatomer subunit gamma-2",
  "term_id": "GO:0005783"
}